{
  "gene_symbol": "MYRF",
  "gene_name": "Myelin regulatory factor",
  "term_id": "GO:0003700",
  "term_label": "DNA-binding transcription factor activity",
  "gene": "UniProtKB:Q9Y2G1"
}